{
  "gene_symbol": "BBS7",
  "gene": "UniProtKB:Q8IWZ6",
  "term_label": "ciliary basal body",
  "gene_name": "Bardet-Biedl syndrome 7 protein",
  "term_id": "GO:0036064"
}